{
  "term_id": "GO:0007030",
  "gene_name": "Transmembrane emp24 domain-containing protein 4",
  "term_label": "Golgi organization",
  "gene": "UniProtKB:Q7Z7H5",
  "gene_symbol": "TMED4"
}